granular component [GO:0001652] (cellular component) Definition: A structure found in the nucleolus, which contains nearly completed preribosomal particles destined for the cytoplasm. Also known as: pars granulosa Relationships: is a type of cellular anatomical structure [GO:0110165]; is part of nucleolus [GO:0005730] References: PMID:10754561